{
  "gene_symbol": "OR7G2",
  "term_label": "plasma membrane",
  "gene": "UniProtKB:Q8NG99",
  "term_id": "GO:0005886",
  "gene_name": "Olfactory receptor 7G2"
}